{
  "term_label": "acetylgalactosaminyltransferase activity",
  "gene_name": "N-acetyl-beta-glucosaminyl-glycoprotein 4-beta-N-acetylgalactosaminyltransferase 1",
  "term_id": "GO:0008376",
  "gene": "UniProtKB:Q76KP1",
  "gene_symbol": "B4GALNT4"
}